{
  "gene": "UniProtKB:Q5VV43",
  "term_id": "GO:0001764",
  "term_label": "neuron migration",
  "gene_symbol": "KIAA0319",
  "gene_name": "Dyslexia-associated protein KIAA0319"
}